positive regulation of digestive system process [GO:0060456] (biological process) Definition: Any process that increases the frequency, rate or extent of a digestive system process, a physical, chemical, or biochemical process carried out by living organisms to break down ingested nutrients into components that may be easily absorbed and directed into metabolism. Sources: GOC:dph, GOC:tb Subtypes: positive regulation of saliva secretion [GO:0046878], positive regulation of hindgut contraction [GO:0060450], positive regulation of gastric acid secretion [GO:0060454], positive regulation of intestinal epithelial structure maintenance [GO:0060731], positive regulation of pancreatic juice secretion [GO:0090187], positive regulation of small intestinal transit [GO:0120058], positive regulation of gastric emptying [GO:0120062], positive regulation of intestinal absorption [GO:1904480], positive regulation of defecation [GO:2000294] Relationships: is a type of regulation of digestive system process [GO:0044058]; is a type of GO:0051240; positively regulates GO:0022600